{
  "term_label": "growth factor activity",
  "gene_symbol": "FGF4",
  "gene": "UniProtKB:P08620",
  "term_id": "GO:0008083",
  "gene_name": "Fibroblast growth factor 4"
}